{
  "gene_name": "Otospiralin",
  "term_id": "UNKNOWN:0001",
  "gene": "UniProtKB:Q8NHW6",
  "term_label": "Unknown molecular function",
  "gene_symbol": "OTOS"
}